{
  "term_label": "RNA polymerase transcription factor SL1 complex",
  "term_id": "GO:0005668",
  "gene": "UniProtKB:Q53T94",
  "gene_symbol": "TAF1B",
  "gene_name": "TATA box-binding protein-associated factor RNA polymerase I subunit B"
}